{
  "term_id": "GO:0047496",
  "gene_symbol": "BICDL1",
  "gene_name": "BICD family-like cargo adapter 1",
  "term_label": "vesicle transport along microtubule",
  "gene": "UniProtKB:Q6ZP65"
}